pristanate-CoA ligase activity [GO:0070251] (molecular function) Also known as: pristanate:CoA ligase (AMP-forming), pristanoyl-CoA ligase activity References: PMID:10198260 Sources: GOC:pde Relationships: is a type of CoA-ligase activity [GO:0016405]; is a type of GO:0016878 Definition: Catalysis of the reaction: ATP + pristanate + CoA = AMP + diphosphate + pristanoyl-CoA.